gibberellic acid mediated signaling pathway [GO:0009740] (biological process) Also known as: GA-signaling, gibberellic acid mediated signalling, gibberellic acid signaling Regulation: regulated by regulation of gibberellic acid mediated signaling pathway [GO:0009937]; negatively regulated by negative regulation of gibberellic acid mediated signaling pathway [GO:0009938]; positively regulated by positive regulation of gibberellic acid mediated signaling pathway [GO:0009939] Subtypes: gibberellic acid mediated signaling pathway, G-alpha-dependent [GO:0042388], GO:0042390 Sources: GOC:sm Relationships: is a type of gibberellin mediated signaling pathway [GO:0010476] Definition: The series of molecular signals mediated by the detection of gibberellic acid.